sensory perception of sweet taste [GO:0050916] (biological process) Definition: The series of events required to receive a sweet taste stimulus, convert it to a molecular signal, and recognize and characterize the signal. This is a neurological process. Also known as: sweet taste perception Regulation: regulated by GO:1904656; negatively regulated by negative regulation of sensory perception of sweet taste [GO:1904657]; positively regulated by GO:1904658 Relationships: is_a GO:0050909 Sources: GOC:ai